{
  "gene": "UniProtKB:P16389",
  "gene_name": "Potassium voltage-gated channel subfamily A member 2",
  "term_label": "juxtaparanode region of axon",
  "gene_symbol": "KCNA2",
  "term_id": "GO:0044224"
}